{
  "gene_name": "Olfactory receptor 8D2",
  "term_id": "GO:0007186",
  "gene": "UniProtKB:Q9GZM6",
  "term_label": "G protein-coupled receptor signaling pathway",
  "gene_symbol": "OR8D2"
}